{
  "term_id": "GO:0007165",
  "term_label": "signal transduction",
  "gene_symbol": "YWHAE",
  "gene_name": "14-3-3 protein epsilon",
  "gene": "UniProtKB:P62258"
}